{
  "gene": "UniProtKB:Q9Y5Y2",
  "term_label": "iron-sulfur cluster binding",
  "gene_name": "Cytosolic Fe-S cluster assembly factor NUBP2",
  "gene_symbol": "NUBP2",
  "term_id": "GO:0051536"
}